{
  "gene_symbol": "GALNT11",
  "term_id": "GO:0005794",
  "gene_name": "Polypeptide N-acetylgalactosaminyltransferase 11",
  "term_label": "Golgi apparatus",
  "gene": "UniProtKB:Q8NCW6"
}